cis-zeatin O-beta-D-glucosyltransferase activity [GO:0050502] (molecular function) Relationships: is a type of UDP-glucosyltransferase activity [GO:0035251] Definition: Catalysis of the reaction: cis-zeatin + UDP-D-glucose = O-beta-D-glucosyl-cis-zeatin + H+ + UDP. Sources: EC:2.4.1.215, RHEA:20681 Also known as: cis-zeatin O-b-D-glucosyltransferase activity, UDP-glucose:cis-zeatin O-beta-D-glucosyltransferase activity, UDPglucose:cis-zeatin O-beta-D-glucosyltransferase activity